cytoplasmic side of cis-Golgi cisternae membrane [GO:0160278] (cellular component) Definition: The membrane leaflet of the cis-Golgi cisternae membrane that faces the cytoplasm and is the site of interactions with cytosolic proteins, including those involved in vesicle budding, membrane tethering, and lipid or protein trafficking. References: PMID:10922460, PMID:34597626, PMID:39331042 Relationships: is a type of cytoplasmic side of membrane [GO:0098562]; is part of GO:1990674 Also known as: cytoplasmic face of cis-Golgi cisternae membrane, cytoplasmic leaflet of cis-Golgi cisternae membrane